hydrogen generation via nitrogenase [GO:0044835] (biological process) Definition: The chemical reactions and pathways resulting in the formation of H2 (dihydrogen) which involve a nitrogenase activity as one of the steps. This process is observed in cyanobacteria. Relationships: is_a hydrogen biosynthetic process [GO:1902422]; has part GO:0016163 References: PMID:22128188 Sources: GOC:mengo_curators